{
  "term_label": "potassium ion import across plasma membrane",
  "gene_symbol": "KCNJ6",
  "term_id": "GO:1990573",
  "gene_name": "G protein-activated inward rectifier potassium channel 2",
  "gene": "UniProtKB:P48051"
}